establishment of mitotic sister chromatid cohesion [GO:0034087] (biological process) Relationships: is a type of establishment of sister chromatid cohesion [GO:0034085]; is a type of mitotic cell cycle process [GO:1903047]; is part of mitotic sister chromatid cohesion [GO:0007064] Definition: The process in which the sister chromatids of a replicated chromosome become joined along the entire length of the chromosome during S phase during a mitotic cell cycle. Sources: GOC:mah